{
  "term_id": "GO:0017158",
  "gene_name": "Synaptotagmin-10",
  "gene_symbol": "SYT10",
  "term_label": "regulation of calcium ion-dependent exocytosis",
  "gene": "UniProtKB:Q6XYQ8"
}